{
  "term_label": "calcium ion binding",
  "gene_name": "Myosin light chain 5",
  "term_id": "GO:0005509",
  "gene": "UniProtKB:Q02045",
  "gene_symbol": "MYL5"
}